{
  "term_id": "GO:0000470",
  "gene": "UniProtKB:P62424",
  "term_label": "maturation of LSU-rRNA",
  "gene_name": "Large ribosomal subunit protein eL8",
  "gene_symbol": "RPL7A"
}